keratinization [GO:0031424] (biological process) Definition: The process in which the cytoplasm of the outermost cells of the vertebrate epidermis is replaced by keratin. Keratinization occurs in the stratum corneum, feathers, hair, claws, nails, hooves, and horns. Relationships: is a type of multicellular organismal process [GO:0032501]; is part of GO:0030216 Sources: GOC:dph, GOC:ebc, GOC:sdb_2009, GOC:tb